{
  "gene_symbol": "PSG9",
  "term_label": "Unknown biological process",
  "term_id": "UNKNOWN:0002",
  "gene_name": "Pregnancy-specific beta-1-glycoprotein 9",
  "gene": "UniProtKB:Q00887"
}